{
  "gene": "UniProtKB:Q96AP0",
  "gene_symbol": "ACD",
  "term_id": "GO:0042162",
  "term_label": "telomeric DNA binding",
  "gene_name": "Adrenocortical dysplasia protein homolog"
}